GTPase-dependent fusogenic activity [GO:0140523] (MF) Definition: A GTPase activity that mediates the joining of two lipid bilayers to form a single membrane. Relationships: is a type of GO:0003924; is a type of fusogenic activity [GO:0140522]; is part of membrane fusion [GO:0061025] Also known as: membrane fusion GTPase activity References: PMID:29663589